{
  "term_id": "UNKNOWN:0001",
  "gene": "UniProtKB:P0DPF7",
  "gene_symbol": "TRBV6-3",
  "gene_name": "T cell receptor beta variable 6-3",
  "term_label": "Unknown molecular function"
}